{
  "term_id": "GO:1990429",
  "term_label": "peroxisomal importomer complex",
  "gene_name": "Peroxisomal membrane protein PEX14",
  "gene_symbol": "PEX14",
  "gene": "UniProtKB:O75381"
}